{
  "term_id": "GO:0030574",
  "gene_symbol": "MMP27",
  "term_label": "collagen catabolic process",
  "gene_name": "Matrix metalloproteinase-27",
  "gene": "UniProtKB:Q9H306"
}